ankyrin-1 complex [GO:0170014] (cellular component) Definition: A complex composed of ANK1, RHCE, RHAG, SLC4A1, EPB42, GYPA, GYPB and AQP1, that functions in the stability and shape of the erythrocyte membrane in human. Relationships: is a type of membrane protein complex [GO:0098796] References: PMID:35835865 Also known as: ankyrin complex, erythrocyte ankyrin-1 complex